pancreatic A cell development [GO:0003322] (BP) Definition: The process whose specific outcome is the progression of a pancreatic A cell over time, from its formation to the mature structure. A pancreatic A cell is a cell in the pancreas that secretes glucagon. Also known as: pancreatic alpha cell development Sources: GOC:dph Relationships: is a type of epithelial cell development [GO:0002064]; is part of GO:0003310